{
  "gene_name": "2'-5'-oligoadenylate synthase 2",
  "gene": "UniProtKB:P29728",
  "gene_symbol": "OAS2",
  "term_id": "GO:0016020",
  "term_label": "membrane"
}